{
  "gene_symbol": "IGKV1D-8",
  "term_id": "GO:0006955",
  "term_label": "immune response",
  "gene": "UniProtKB:A0A087WSZ0",
  "gene_name": "Immunoglobulin kappa variable 1D-8"
}